ABC-type sodium transporter activity [GO:0140679] (molecular function) Definition: Enables the transfer of a solute or solutes from one side of a membrane to the other according to the reaction: ATP + H2O + Na(in) = ADP + phosphate + Na(out). References: PMID:9106203 Relationships: is a type of GO:0015081; is a type of GO:0019829; is a type of ABC-type transporter activity [GO:0140359]